2-oxoglutarate decarboxylation to succinyl-CoA [GO:0120551] (biological process) Also known as: 2-ketoglutarate dehydrogenase system, 2-oxoglutarate dehydrogenase system, 2alpha-ketoglutarate dehydrogenase system Definition: The chemical reactions and pathways resulting in the formation of succinyl-CoA from 2-oxoglutarate.  In most organisms, this pathway is part of the TCA cycle and comprises a series of three reactions carried out by a multisubunit complex called the '2-oxoglutarate dehydrogenase complex', even though 2-oxoglutarate dehydrogenase activity describes only one of those reactions. The combination of the three reactions can be summarized as: 2-oxoglutarate + coenzyme A + NAD+ -> succinyl-CoA + CO2 + NADH. Sources: MetaCyc:PWY-5084 Relationships: is a type of 2-oxoglutarate metabolic process [GO:0006103]; is a type of succinyl-CoA biosynthetic process [GO:1901290]; is part of tricarboxylic acid cycle [GO:0006099]